detection of chemical stimulus involved in sensory perception of umami taste [GO:0046535] (biological process) Also known as: perception of umami taste, detection of chemical stimulus, perception of umami taste, sensory transduction of chemical stimulus, sensory detection of chemical stimulus during perception of umami taste, sensory detection of umami taste, sensory transduction of chemical stimulus during perception of umami taste, sensory transduction of umami taste, umami taste detection Relationships: is a type of detection of chemical stimulus involved in sensory perception of taste [GO:0050912]; is part of sensory perception of umami taste [GO:0050917] Definition: The series of events required for a umami taste stimulus to be received and converted to a molecular signal. Umami taste is the savory taste of meats and other foods that are rich in glutamates. References: PMID:11894099 Sources: GOC:ai, GOC:dos